{
  "gene_symbol": "RPA2",
  "gene_name": "Replication protein A 32 kDa subunit",
  "term_id": "GO:0000724",
  "term_label": "double-strand break repair via homologous recombination",
  "gene": "UniProtKB:P15927"
}